{
  "gene_name": "Nucleolar protein 9",
  "term_label": "endonucleolytic cleavage in ITS1 to separate SSU-rRNA from 5.8S rRNA and LSU-rRNA from tricistronic rRNA transcript (SSU-rRNA, 5.8S rRNA, LSU-rRNA)",
  "gene_symbol": "NOP9",
  "gene": "UniProtKB:Q86U38",
  "term_id": "GO:0000447"
}